coronary sinus valve formation [GO:0003191] (biological process) Relationships: is a type of heart valve formation [GO:0003188]; is part of coronary sinus valve morphogenesis [GO:0003182] Sources: GOC:mtg_heart Definition: The developmental process pertaining to the initial formation of the coronary sinus valve from unspecified parts. This process begins with the specific processes that contribute to the appearance of the discrete structure and ends when the structural rudiment is recognizable.